{
  "term_id": "GO:0019814",
  "gene_symbol": "IGLV8-61",
  "gene": "UniProtKB:A0A075B6I0",
  "gene_name": "Immunoglobulin lambda variable 8-61",
  "term_label": "immunoglobulin complex"
}